skeletal muscle satellite cell fate specification [GO:0014817] (biological process) References: PMID:16607119 Sources: GOC:ef, GOC:mtg_muscle Relationships: is a type of cell fate specification [GO:0001708]; is part of skeletal muscle satellite cell commitment [GO:0014813] Definition: The process in which a cell becomes capable of differentiating autonomously into a skeletal muscle satellite cell in an environment that is neutral with respect to the developmental pathway. Upon specification, the cell fate can be reversed.